{
  "gene_name": "Transducin-like enhancer protein 3",
  "gene": "UniProtKB:Q04726",
  "term_label": "transcription corepressor activity",
  "gene_symbol": "TLE3",
  "term_id": "GO:0003714"
}